{
  "gene": "UniProtKB:Q9NVV0",
  "term_label": "release of sequestered calcium ion into cytosol by sarcoplasmic reticulum",
  "gene_name": "Trimeric intracellular cation channel type B",
  "gene_symbol": "TMEM38B",
  "term_id": "GO:0014808"
}